{
  "term_id": "UNKNOWN:0003",
  "gene_name": "Oxidoreductase NAD-binding domain-containing protein 1",
  "term_label": "Unknown cellular component",
  "gene_symbol": "OXNAD1",
  "gene": "UniProtKB:Q96HP4"
}